regulation of error-prone translesion synthesis [GO:1904331] (biological process) Definition: Any process that modulates the frequency, rate or extent of error-prone translesion synthesis. Also known as: regulation of mutagenic PRR, regulation of error-prone postreplication DNA repair, regulation of mutagenic postreplication DNA repair Subtypes: negative regulation of error-prone translesion synthesis [GO:1904332], positive regulation of error-prone translesion synthesis [GO:1904333] References: PMID:22761594 Sources: GOC:TermGenie, GOC:kmv, GO_REF:0000058 Relationships: is a type of regulation of cellular response to stress [GO:0080135]; is a type of GO:2000278; regulates error-prone translesion synthesis [GO:0042276]